{
  "term_label": "Unknown cellular component",
  "gene_name": "DEP domain-containing protein 7",
  "gene_symbol": "DEPDC7",
  "gene": "UniProtKB:Q96QD5",
  "term_id": "UNKNOWN:0003"
}